lens epithelial cell proliferation [GO:0097166] (biological process) Regulation: regulated by regulation of lens epithelial cell proliferation [GO:2001109]; negatively regulated by negative regulation of lens epithelial cell proliferation [GO:2001110]; positively regulated by positive regulation of lens epithelial cell proliferation [GO:2001111] Relationships: is a type of epithelial cell proliferation [GO:0050673]; BFO_0000050 lens development in camera-type eye [GO:0002088] Definition: The multiplication or reproduction of lens epithelial cells, resulting in the expansion of a cell population. Lens epithelial cells make up the lens epithelium, which is located in the anterior portion of the lens between the lens capsule and the lens fibers and is a simple cuboidal epithelium. The epithelial cells of the lens regulate most of the homeostatic functions of the lens such as osmolarity and liquid volume. The lens epithelial cells also serve as the progenitors for new lens fibers. The lens epithelium constantly lays down fibers in the embryo, fetus, infant, and adult, and continues to lay down fibers for lifelong growth. References: PMID:18423449 Sources: CL:0002224, GOC:yaf, Wikipedia:Lens_%28anatomy%29#Lens_epithelium